{
  "gene_name": "Serine protease 38",
  "gene_symbol": "PRSS38",
  "gene": "UniProtKB:A1L453",
  "term_label": "serine-type endopeptidase activity",
  "term_id": "GO:0004252"
}